positive regulation of receptor-mediated endocytosis involved in cholesterol transport [GO:1905602] (biological process) References: PMID:22848640 Sources: GOC:BHF, GOC:TermGenie, GOC:nc, GO_REF:0000058 Definition: Any process that activates or increases the frequency, rate or extent of receptor-mediated endocytosis involved in cholesterol transport. Relationships: is a type of positive regulation of intracellular cholesterol transport [GO:0032385]; is_a positive regulation of receptor-mediated endocytosis [GO:0048260]; is a type of GO:1905600; positively regulates receptor-mediated endocytosis involved in cholesterol transport [GO:0090118] Also known as: up regulation of receptor-mediated endocytosis involved in cholesterol transport, up-regulation of receptor-mediated endocytosis involved in cholesterol transport, upregulation of receptor-mediated endocytosis involved in cholesterol transport, activation of receptor-mediated endocytosis involved in cholesterol transport, activation of receptor-mediated endocytosis of LDL, activation of receptor-mediated endocytosis involved in intracellular cholesterol transport, activation of receptor-mediated endocytosis of low-density lipoprotein involved in cholesterol transport, activation of receptor-mediated endocytosis of low-density lipoprotein particle involved in cholesterol transport, positive regulation of receptor-mediated endocytosis involved in intracellular cholesterol transport, positive regulation of receptor-mediated endocytosis of LDL, positive regulation of receptor-mediated endocytosis of low-density lipoprotein involved in cholesterol transport, positive regulation of receptor-mediated endocytosis of low-density lipoprotein particle involved in cholesterol transport, up regulation of receptor-mediated endocytosis involved in intracellular cholesterol transport, up regulation of receptor-mediated endocytosis of LDL, up regulation of receptor-mediated endocytosis of low-density lipoprotein involved in cholesterol transport, up regulation of receptor-mediated endocytosis of low-density lipoprotein particle involved in cholesterol transport, up-regulation of receptor-mediated endocytosis involved in intracellular cholesterol transport, up-regulation of receptor-mediated endocytosis of LDL, up-regulation of receptor-mediated endocytosis of low-density lipoprotein involved in cholesterol transport, up-regulation of receptor-mediated endocytosis of low-density lipoprotein particle involved in cholesterol transport, upregulation of receptor-mediated endocytosis involved in intracellular cholesterol transport, upregulation of receptor-mediated endocytosis of LDL, upregulation of receptor-mediated endocytosis of low-density lipoprotein involved in cholesterol transport, upregulation of receptor-mediated endocytosis of low-density lipoprotein particle involved in cholesterol transport